IgE binding [GO:0019863] (molecular function) Relationships: is a type of GO:0019865 Definition: Binding to an immunoglobulin of the IgE isotype. Sources: GOC:add, ISBN:0781735149